{
  "term_id": "GO:0005739",
  "gene": "UniProtKB:Q4G176",
  "term_label": "mitochondrion",
  "gene_name": "Malonate--CoA ligase ACSF3, mitochondrial",
  "gene_symbol": "ACSF3"
}